{
  "term_id": "GO:0006357",
  "gene": "UniProtKB:P51815",
  "term_label": "regulation of transcription by RNA polymerase II",
  "gene_name": "Zinc finger protein 75D",
  "gene_symbol": "ZNF75D"
}